{
  "term_label": "Unknown biological process",
  "gene": "UniProtKB:Q86VM9",
  "term_id": "UNKNOWN:0002",
  "gene_symbol": "ZC3H18",
  "gene_name": "Zinc finger CCCH domain-containing protein 18"
}